{
  "gene_symbol": "E2F2",
  "gene": "UniProtKB:Q14209",
  "term_label": "RNA polymerase II cis-regulatory region sequence-specific DNA binding",
  "term_id": "GO:0000978",
  "gene_name": "Transcription factor E2F2"
}